{
  "term_label": "Unknown biological process",
  "gene_symbol": "CEP85L",
  "term_id": "UNKNOWN:0002",
  "gene": "UniProtKB:Q5SZL2",
  "gene_name": "Centrosomal protein of 85 kDa-like"
}